{
  "term_label": "Unknown biological process",
  "gene": "UniProtKB:Q6S8J7",
  "gene_name": "POTE ankyrin domain family member A",
  "term_id": "UNKNOWN:0002",
  "gene_symbol": "POTEA"
}